{
  "term_id": "GO:0005743",
  "gene_name": "ADP_ATP translocase 3",
  "gene_symbol": "SLC25A6",
  "term_label": "mitochondrial inner membrane",
  "gene": "UniProtKB:P12236"
}